symbiont-mediated actin polymerization-dependent cell-to-cell migration in host [GO:0070360] (biological process) Also known as: actin polymerization-dependent cell migration in host, actin polymerization-dependent cell-to-cell migration in host, actin polymerization-dependent cell motility involved in migration of symbiont in host, migration of symbiont within host by polymerization of host actin Definition: The directional movement of an organism, usually a bacterial cell, from one place to another within its host organism, by a process involving continuous polymerization of actin at one pole of the symbiont cell. Some bacteria use host actin for migration from cell to cell. The host is defined as the larger of the organisms involved in a symbiotic interaction. References: PMID:15773977, PMID:15981456, PMID:26021574, PMID:27997855, PMID:35285700 Sources: GOC:jl, GOC:mah Relationships: is a type of actin polymerization-dependent cell motility [GO:0070358]; is a type of symbiont-mediated cell-to-cell migration in host [GO:0106259]